{
  "gene_symbol": "PROKR1",
  "gene": "UniProtKB:Q8TCW9",
  "term_label": "circadian rhythm",
  "term_id": "GO:0007623",
  "gene_name": "Prokineticin receptor 1"
}